{
  "term_id": "GO:0001228",
  "gene": "UniProtKB:Q7Z6R9",
  "gene_symbol": "TFAP2D",
  "term_label": "DNA-binding transcription activator activity, RNA polymerase II-specific",
  "gene_name": "Transcription factor AP-2-delta"
}